protein dehydration [GO:0018249] (biological process) Relationships: is a type of GO:0036211 Definition: The removal of a water group from a protein amino acid. Subtypes: peptidyl-tyrosine dehydrogenation [GO:0018251] Also known as: protein amino acid dehydration Sources: GOC:ai